{
  "gene_name": "Tubulin epsilon chain",
  "gene_symbol": "TUBE1",
  "gene": "UniProtKB:Q9UJT0",
  "term_label": "microtubule cytoskeleton organization",
  "term_id": "GO:0000226"
}